positive regulation of lipoprotein transport [GO:0140077] (biological process) References: PMID:26501192 Sources: GOC:BHF, GOC:BHF_miRNA, GOC:RPH Definition: Any process that activates or increases the rate or extent of lipoprotein transport. Relationships: is a type of positive regulation of protein transport [GO:0051222]; is a type of GO:0140075; positively regulates GO:0042953